{
  "gene": "UniProtKB:Q9H2X9",
  "gene_symbol": "SLC12A5",
  "gene_name": "Solute carrier family 12 member 5",
  "term_id": "GO:0055075",
  "term_label": "potassium ion homeostasis"
}